rhombomere 7 morphogenesis [GO:0021671] (biological process) Relationships: is a type of rhombomere morphogenesis [GO:0021593]; is part of rhombomere 7 development [GO:0021573] Sources: GOC:cls, GOC:curators, GOC:dgh, GOC:dph, GOC:jid Definition: The process in which the anatomical structure of rhombomere 7 is generated and organized. Rhombomeres are transverse segments of the developing rhombencephalon. Rhombomeres are lineage restricted, express different genes from one another, and adopt different developmental fates. Rhombomeres are numbered in an anterior to posterior order.